{
  "gene": "UniProtKB:Q6TDU7",
  "gene_name": "Dynein axonemal intermediate chain 7",
  "gene_symbol": "DNAI7",
  "term_id": "GO:0005930",
  "term_label": "axoneme"
}